{
  "term_label": "Unknown cellular component",
  "gene_symbol": "APOBEC4",
  "gene_name": "Putative C-U-editing enzyme APOBEC-4",
  "gene": "UniProtKB:Q8WW27",
  "term_id": "UNKNOWN:0003"
}